{
  "term_id": "GO:0004865",
  "gene_symbol": "PPP1R14D",
  "gene_name": "Protein phosphatase 1 regulatory subunit 14D",
  "gene": "UniProtKB:Q9NXH3",
  "term_label": "protein serine/threonine phosphatase inhibitor activity"
}